heteroglycan alpha-mannosyltransferase activity [GO:0047264] (molecular function) Relationships: is a type of mannosyltransferase activity [GO:0000030] Definition: Catalysis of the reaction: heteroglycan + GDP-mannose = alpha-D-mannosylheteroglycan + GDP. 1,2- and 1,3-mannosyl bonds are formed. Sources: EC:2.4.1.48 Also known as: heteropolysaccharide alpha-mannosyltransferase activity, GDP mannose alpha-mannosyltransferase activity, GDP-mannose:heteroglycan 2-(or 3-)-alpha-D-mannosyltransferase activity, guanosine diphosphomannose-heteroglycan alpha-mannosyltransferase activity